{
  "gene_name": "NBAS subunit of NRZ tethering complex",
  "gene": "UniProtKB:A2RRP1",
  "term_label": "SNARE binding",
  "term_id": "GO:0000149",
  "gene_symbol": "NBAS"
}